{
  "term_id": "GO:0046103",
  "gene_symbol": "ADA2",
  "term_label": "inosine biosynthetic process",
  "gene": "UniProtKB:Q9NZK5",
  "gene_name": "Adenosine deaminase 2"
}